{
  "gene_symbol": "FDXR",
  "term_id": "GO:0005739",
  "term_label": "mitochondrion",
  "gene": "UniProtKB:P22570",
  "gene_name": "NADPH:adrenodoxin oxidoreductase, mitochondrial"
}